{
  "term_id": "GO:0051087",
  "gene_symbol": "FNIP2",
  "term_label": "protein-folding chaperone binding",
  "gene_name": "Folliculin-interacting protein 2",
  "gene": "UniProtKB:Q9P278"
}